neurofilament cytoskeleton [GO:0060053] (cellular component) Definition: Intermediate filament cytoskeletal structure that is made up of neurofilaments. Neurofilaments are specialized intermediate filaments found in neurons. Sources: GOC:dph Relationships: is a type of intermediate filament cytoskeleton [GO:0045111]; has part neurofilament [GO:0005883]